{
  "term_label": "spermatogenesis",
  "term_id": "GO:0007283",
  "gene": "UniProtKB:Q8TC59",
  "gene_symbol": "PIWIL2",
  "gene_name": "Piwi-like protein 2"
}